{
  "term_label": "oxidative RNA demethylation",
  "gene": "UniProtKB:Q13686",
  "term_id": "GO:0035513",
  "gene_symbol": "ALKBH1",
  "gene_name": "Nucleic acid dioxygenase ALKBH1"
}